{
  "term_label": "JUN kinase kinase kinase activity",
  "term_id": "GO:0004706",
  "gene": "UniProtKB:Q16584",
  "gene_symbol": "MAP3K11",
  "gene_name": "Mitogen-activated protein kinase kinase kinase 11"
}